{
  "gene": "UniProtKB:Q96SB8",
  "term_label": "Smc5-Smc6 complex",
  "gene_name": "Structural maintenance of chromosomes protein 6",
  "gene_symbol": "SMC6",
  "term_id": "GO:0030915"
}